{
  "gene": "UniProtKB:Q9UIX4",
  "term_id": "GO:0071805",
  "gene_name": "Potassium voltage-gated channel subfamily G member 1",
  "term_label": "potassium ion transmembrane transport",
  "gene_symbol": "KCNG1"
}